specification of animal organ position [GO:0010159] (biological process) Sources: GOC:curators Relationships: is a type of regionalization [GO:0003002]; is part of animal organ morphogenesis [GO:0009887] Definition: The regionalization process in which information that determines the correct position at which animal organ primordia are formed is generated and perceived resulting in correct positioning of the new animal organ.